symbiont-mediated disruption of host chloroplast [GO:0033656] (BP) Also known as: disruption by symbiont of host chloroplast, modification by symbiont of host chloroplast Relationships: is a type of symbiont-mediated disruption of host cellular anatomical structure [GO:0052008] Sources: GOC:pamgo_curators Definition: The process in which an organism effects a change that impairs the structure or function of the host chloroplast. The host is defined as the larger of the organisms involved in a symbiotic interaction.